{
  "term_label": "extracellular space",
  "gene_name": "Bone morphogenetic protein 2",
  "gene_symbol": "BMP2",
  "term_id": "GO:0005615",
  "gene": "UniProtKB:P12643"
}